nucleotidase activity [GO:0008252] (molecular function) Sources: RHEA:22140 Subtypes: GO:0008253, 3'-nucleotidase activity [GO:0008254], 3'(2'),5'-bisphosphate nucleotidase activity [GO:0008441] Also known as: NSP I, NSP II, acid nucleotidase activity, deoxyinosine-activated nucleotidase (DIAN), deoxyribonucleoside-activated nucleotidase (DAN), nucleotide phosphohydrolase activity, nucleotide-specific phosphatase activity Definition: Catalysis of the reaction: a nucleotide + H2O = a nucleoside + phosphate. Relationships: is a type of phosphatase activity [GO:0016791]